cell plate formation involved in plant-type cell wall biogenesis [GO:0009920] (BP) Relationships: is a type of GO:0000919; is a type of mitotic cell cycle process [GO:1903047]; is part of plant-type cell wall biogenesis [GO:0009832]; is part of GO:0061640; is part of mitotic nuclear division [GO:0140014] Sources: GOC:mtg_sensu, GOC:tb, ISBN:0879015322 Also known as: cell plate formation involved in cellulose and pectin-containing cell wall biogenesis Definition: The cell cycle process in which the cell plate is formed at the equator of the spindle in the dividing cells during early telophase. An example of this is found in Arabidopsis thaliana.